cell wall biogenesis [GO:0042546] (biological process) Subtypes: fungal-type cell wall biogenesis [GO:0009272], peptidoglycan-based cell wall biogenesis [GO:0009273], plant-type cell wall biogenesis [GO:0009832], spore wall biogenesis [GO:0070590] Sources: GOC:jl, GOC:mah, GOC:mtg_sensu, ISBN:0198506732 Relationships: is a type of cellular component biogenesis [GO:0044085]; is a type of cell wall organization or biogenesis [GO:0071554] Definition: A cellular process that results in the biosynthesis of constituent macromolecules, assembly, and arrangement of constituent parts of a cell wall. Includes biosynthesis of constituent macromolecules, such as proteins and polysaccharides, and those macromolecular modifications that are involved in synthesis or assembly of the cellular component. A cell wall is the rigid or semi-rigid envelope lying outside the cell membrane of plant, fungal and most prokaryotic cells, maintaining their shape and protecting them from osmotic lysis. Also known as: cell wall assembly